negative regulation of vitellogenesis [GO:1903187] (biological process) Definition: Any process that stops, prevents or reduces the frequency, rate or extent of vitellogenesis. References: PMID:19467235 Sources: GOC:TermGenie, GOC:mr, GO_REF:0000058 Also known as: down regulation of vitellogenesis, down regulation of yolk production, down-regulation of vitellogenesis, down-regulation of yolk production, downregulation of vitellogenesis, downregulation of yolk production, negative regulation of yolk production, inhibition of vitellogenesis, inhibition of yolk production Relationships: is a type of negative regulation of cellular component organization [GO:0051129]; is a type of negative regulation of multicellular organismal process [GO:0051241]; is a type of regulation of vitellogenesis [GO:1903186]; negatively regulates vitellogenesis [GO:0007296]